{
  "term_id": "GO:0005739",
  "term_label": "mitochondrion",
  "gene_name": "Glutamate dehydrogenase 2, mitochondrial",
  "gene": "UniProtKB:P49448",
  "gene_symbol": "GLUD2"
}